{
  "gene_name": "Alpha-1,6-mannosyl-glycoprotein 2-beta-N-acetylglucosaminyltransferase",
  "gene_symbol": "MGAT2",
  "term_id": "GO:0006487",
  "term_label": "protein N-linked glycosylation",
  "gene": "UniProtKB:Q10469"
}